acetyl-CoA biosynthetic process from pantothenate [GO:1990181] (biological process) References: PMID:23091701 Sources: GOC:mah Relationships: is a type of acetyl-CoA biosynthetic process [GO:0006085]; is a type of pantothenate metabolic process [GO:0015939] Also known as: acetyl-CoA anabolism from pantothenate, acetyl-CoA formation from pantothenate, acetyl-CoA synthesis from pantothenate Definition: The chemical reactions and pathways resulting in the formation of acetyl-CoA from pantothenate via phosphopantothenate and CoA.